{
  "term_id": "GO:0009897",
  "gene_name": "Tumor necrosis factor receptor superfamily member 13C",
  "gene_symbol": "TNFRSF13C",
  "term_label": "external side of plasma membrane",
  "gene": "UniProtKB:Q96RJ3"
}